{
  "gene": "UniProtKB:P00709",
  "gene_name": "Alpha-lactalbumin",
  "gene_symbol": "LALBA",
  "term_label": "defense response to Gram-positive bacterium",
  "term_id": "GO:0050830"
}